{
  "term_id": "GO:0009931",
  "gene_name": "MAP kinase-activated protein kinase 3",
  "gene_symbol": "MAPKAPK3",
  "term_label": "calcium-dependent protein serine/threonine kinase activity",
  "gene": "UniProtKB:Q16644"
}